{
  "term_label": "peptide hormone binding",
  "gene_symbol": "GHR",
  "gene": "UniProtKB:P10912",
  "term_id": "GO:0017046",
  "gene_name": "Growth hormone receptor"
}